{
  "term_label": "lamellipodium assembly",
  "gene_symbol": "CYFIP1",
  "term_id": "GO:0030032",
  "gene": "UniProtKB:Q7L576",
  "gene_name": "Cytoplasmic FMR1-interacting protein 1"
}